{
  "term_label": "extracellular space",
  "gene_symbol": "DKKL1",
  "gene_name": "Dickkopf-like protein 1",
  "gene": "UniProtKB:Q9UK85",
  "term_id": "GO:0005615"
}